{
  "gene_name": "Cilia- and flagella-associated protein 221",
  "gene": "UniProtKB:Q4G0U5",
  "term_id": "UNKNOWN:0001",
  "term_label": "Unknown molecular function",
  "gene_symbol": "CFAP221"
}